{
  "gene_name": "Glycogen synthase kinase-3 beta",
  "term_id": "GO:0008286",
  "gene_symbol": "GSK3B",
  "term_label": "insulin receptor signaling pathway",
  "gene": "UniProtKB:P49841"
}